{
  "term_label": "cilium assembly",
  "gene": "UniProtKB:Q8WXW3",
  "term_id": "GO:0060271",
  "gene_name": "Progesterone-induced-blocking factor 1",
  "gene_symbol": "PIBF1"
}